{
  "term_label": "Unknown cellular component",
  "gene_symbol": "Q8IZM0",
  "term_id": "UNKNOWN:0003",
  "gene_name": "Putative CNGA1-overlapping antisense gene protein",
  "gene": "UniProtKB:Q8IZM0"
}